{
  "gene_symbol": "MFSD12",
  "term_id": "GO:1903712",
  "gene_name": "Major facilitator superfamily domain-containing protein 12",
  "gene": "UniProtKB:Q6NUT3",
  "term_label": "cysteine transmembrane transport"
}